{
  "gene_name": "Steroid receptor RNA activator 1",
  "term_label": "Unknown biological process",
  "gene_symbol": "SRA1",
  "gene": "UniProtKB:Q9HD15",
  "term_id": "UNKNOWN:0002"
}